dicarboxylic acid catabolic process [GO:0043649] (biological process) Relationships: is a type of dicarboxylic acid metabolic process [GO:0043648]; is a type of carboxylic acid catabolic process [GO:0046395] Sources: ISBN:0198506732 Also known as: dicarboxylate catabolic process, dicarboxylate catabolism, dicarboxylic acid breakdown, dicarboxylic acid catabolism, dicarboxylic acid degradation Definition: The chemical reactions and pathways resulting in the breakdown of dicarboxylic acids, any organic acid containing two carboxyl (-COOH) groups. Subtypes: L-aspartate catabolic process [GO:0006533], L-glutamate catabolic process [GO:0006538], 10-formyltetrahydrofolate catabolic process [GO:0009258], L-asparagine biosynthetic process from oxaloacetate [GO:0019266], GO:0019554, aldaric acid catabolic process [GO:0019579], GO:0033611, quinolinate catabolic process [GO:0034213], folic acid catabolic process [GO:0046657], GO:0090410, actinorhodin catabolic process [GO:1901111], 5,6,7,8-tetrahydromethanopterin catabolic process [GO:1901284], prephenate(2-) catabolic process [GO:1901746]